{
  "gene_symbol": "ZNF460",
  "gene": "UniProtKB:Q14592",
  "term_id": "UNKNOWN:0003",
  "term_label": "Unknown cellular component",
  "gene_name": "Zinc finger protein 460"
}